{
  "gene_name": "Follistatin",
  "gene_symbol": "FST",
  "term_label": "cell differentiation",
  "term_id": "GO:0030154",
  "gene": "UniProtKB:P19883"
}